methylcytosine to 5-glyceryl-methylcytosine dioxygenase activity [GO:0120204] (molecular function) Definition: Catalysis of the reaction: methylcytosine + L-ascorbate + O2 = 5-glyceryl-methylcytosine + glyoxylate + CO2. References: PMID:31043749 Relationships: is a type of oxidoreductase activity, acting on paired donors, with incorporation or reduction of molecular oxygen [GO:0016705]